{
  "term_id": "UNKNOWN:0003",
  "gene_symbol": "MMTAG2",
  "gene": "UniProtKB:Q9BU76",
  "gene_name": "Multiple myeloma tumor-associated protein 2",
  "term_label": "Unknown cellular component"
}